{
  "gene_symbol": "AURKC",
  "term_id": "UNKNOWN:0001",
  "term_label": "Unknown molecular function",
  "gene": "UniProtKB:Q9UQB9",
  "gene_name": "Aurora kinase C"
}